ModE complex [GO:1990198] (cellular component) Also known as: ModE dimer Relationships: is a type of transcription regulator complex [GO:0005667]; is part of cytosol [GO:0005829] Definition: A dimeric protein complex containing two ModE subunits. Binds directly to DNA to regulate transcription, and is involved in (positively and negatively) regulating various aspects of molybdenum metabolism. References: PMID:12581638 Sources: GOC:bhm